{
  "gene_name": "Matrix-remodeling-associated protein 5",
  "term_label": "Unknown molecular function",
  "gene": "UniProtKB:Q9NR99",
  "gene_symbol": "MXRA5",
  "term_id": "UNKNOWN:0001"
}